{
  "gene_symbol": "CALHM6",
  "term_label": "monoatomic cation channel activity",
  "term_id": "GO:0005261",
  "gene_name": "Calcium homeostasis modulator protein 6",
  "gene": "UniProtKB:Q5R3K3"
}